{
  "gene_name": "Transducin beta-like protein 2",
  "gene_symbol": "TBL2",
  "term_label": "Unknown molecular function",
  "term_id": "UNKNOWN:0001",
  "gene": "UniProtKB:Q9Y4P3"
}